{
  "term_id": "GO:0044818",
  "term_label": "mitotic G2/M transition checkpoint",
  "gene_symbol": "NABP2",
  "gene": "UniProtKB:Q9BQ15",
  "gene_name": "SOSS complex subunit B1"
}